{
  "gene_symbol": "LHX2",
  "term_id": "GO:0000977",
  "gene_name": "LIM_homeobox protein Lhx2",
  "gene": "UniProtKB:P50458",
  "term_label": "RNA polymerase II transcription regulatory region sequence-specific DNA binding"
}